{
  "gene_symbol": "GFRA3",
  "term_id": "GO:0043235",
  "gene": "UniProtKB:O60609",
  "gene_name": "GDNF family receptor alpha-3",
  "term_label": "receptor complex"
}